{
  "term_label": "cytoplasm",
  "term_id": "GO:0005737",
  "gene_name": "TPT1-like protein",
  "gene_symbol": "Q56UQ5",
  "gene": "UniProtKB:Q56UQ5"
}